{
  "term_label": "sodium:proton antiporter activity",
  "gene_symbol": "SLC9A5",
  "gene": "UniProtKB:Q14940",
  "term_id": "GO:0015385",
  "gene_name": "Sodium_hydrogen exchanger 5"
}